G-quadruplex RNA binding [GO:0002151] (molecular function) Also known as: G quartet binding, G-quartet binding, G quadruplex binding, G quartet RNA binding Note: The structures of RNA and DNA G quartets differ regarding sugar conformation so that a protein binding to the RNA structure might not bind to the DNA structure. Definition: Binding to a G-quadruplex RNA structure, in which groups of four guanines adopt a flat, cyclic hydrogen-bonding arrangement known as a guanine tetrad. References: PMID:18294969, PMID:18568163, PMID:19330720 Relationships: is a type of RNA binding [GO:0003723]